{
  "gene": "UniProtKB:Q15363",
  "gene_name": "Transmembrane emp24 domain-containing protein 2",
  "gene_symbol": "TMED2",
  "term_label": "Golgi organization",
  "term_id": "GO:0007030"
}